{
  "gene_symbol": "SERPINE2",
  "term_id": "GO:0004867",
  "gene_name": "Glia-derived nexin",
  "term_label": "serine-type endopeptidase inhibitor activity",
  "gene": "UniProtKB:P07093"
}